gibberellic acid mediated signaling pathway, G-alpha-dependent [GO:0042388] (biological process) Also known as: gibberellic acid mediated signalling, G-alpha-dependent Definition: The series of molecular signals mediated by the detection of gibberellic acid and dependent on the coupling of the alpha subunit of G proteins to the hormone receptors. Relationships: is a type of gibberellic acid mediated signaling pathway [GO:0009740] References: PMID:11027362 Sources: GOC:pj